{
  "term_label": "cytokine activity",
  "term_id": "GO:0005125",
  "gene_symbol": "IL1B",
  "gene_name": "Interleukin-1 beta",
  "gene": "UniProtKB:P01584"
}